{
  "term_label": "Unknown molecular function",
  "gene_name": "S-adenosylhomocysteine hydrolase-like protein 1",
  "gene": "UniProtKB:O43865",
  "gene_symbol": "AHCYL1",
  "term_id": "UNKNOWN:0001"
}